vitamin B6 metabolic process [GO:0042816] (biological process) Definition: The chemical reactions and pathways involving any of the vitamin B6 compounds: pyridoxal, pyridoxamine and pyridoxine and the active form, pyridoxal phosphate. References: PMID:30037155, PMID:30671974 Sources: GOC:jl Relationships: is a type of GO:0072524 Also known as: vitamin B6 metabolism Subtypes: GO:0008614, pyridoxal metabolic process [GO:0042817], pyridoxamine metabolic process [GO:0042818], vitamin B6 biosynthetic process [GO:0042819], vitamin B6 catabolic process [GO:0042820], pyridoxal phosphate metabolic process [GO:0042822]